{
  "term_label": "cytoplasm",
  "gene_symbol": "PRAMEF33",
  "gene": "UniProtKB:A0A0G2JMD5",
  "gene_name": "PRAME family member 33",
  "term_id": "GO:0005737"
}